{
  "term_id": "UNKNOWN:0003",
  "gene": "UniProtKB:Q5T319",
  "term_label": "Unknown cellular component",
  "gene_symbol": "FAM182B",
  "gene_name": "Protein FAM182B"
}